{
  "gene": "UniProtKB:A6NC05",
  "term_label": "Unknown biological process",
  "gene_symbol": "C5orf63",
  "term_id": "UNKNOWN:0002",
  "gene_name": "Glutaredoxin-like protein C5orf63"
}